{
  "term_label": "G protein-coupled receptor kinase activity",
  "gene": "UniProtKB:P43250",
  "gene_symbol": "GRK6",
  "term_id": "GO:0004703",
  "gene_name": "G protein-coupled receptor kinase 6"
}